{
  "term_id": "GO:0005634",
  "gene_symbol": "LMX1A",
  "term_label": "nucleus",
  "gene": "UniProtKB:Q8TE12",
  "gene_name": "LIM homeobox transcription factor 1-alpha"
}